DNA synthesis involved in double-strand break repair via single-strand annealing [GO:0043151] (biological process) Also known as: DNA synthesis during double-strand break repair via single-strand annealing Relationships: is a type of DNA synthesis involved in DNA repair [GO:0000731]; is part of double-strand break repair via single-strand annealing [GO:0045002] Definition: The synthesis of DNA that contributes to the process of double-strand break repair via single-strand annealing. Sources: GOC:go_curators